cell adhesion involved in dendrite retrograde extension [GO:0003394] (biological process) Definition: The attachment of a cell, either to another cell or to an underlying substrate such as the extracellular matrix that contributes to the process of retrograde extension of a dendrite. Sources: GOC:ascb_2009, GOC:dph, GOC:tb Subtypes: cell adhesion involved in amphid sensory organ dendrite retrograde extension [GO:0003396] Relationships: is a type of cell adhesion involved in retrograde extension [GO:0003392]; is part of dendrite development by retrograde extension [GO:0003390]